{
  "term_id": "UNKNOWN:0003",
  "gene_name": "G antigen 2A",
  "gene_symbol": "GAGE2A",
  "term_label": "Unknown cellular component",
  "gene": "UniProtKB:Q6NT46"
}